{
  "gene_name": "Phospholipase A2",
  "gene": "UniProtKB:P04054",
  "term_id": "GO:0046470",
  "gene_symbol": "PLA2G1B",
  "term_label": "phosphatidylcholine metabolic process"
}